{
  "gene_symbol": "BCCIP",
  "term_id": "UNKNOWN:0002",
  "gene_name": "BRCA2 and CDKN1A-interacting protein",
  "term_label": "Unknown biological process",
  "gene": "UniProtKB:Q9P287"
}